{
  "gene_symbol": "ST8SIA3",
  "gene": "UniProtKB:O43173",
  "term_id": "GO:0003828",
  "term_label": "alpha-N-acetylneuraminate alpha-2,8-sialyltransferase activity",
  "gene_name": "Sia-alpha-2,3-Gal-beta-1,4-GlcNAc-R:alpha 2,8-sialyltransferase"
}